{
  "gene_symbol": "RAB6D",
  "gene_name": "Ras-related protein Rab-6D",
  "term_label": "retrograde transport, endosome to Golgi",
  "term_id": "GO:0042147",
  "gene": "UniProtKB:Q53S08"
}